negative regulation of Wnt signaling pathway, planar cell polarity pathway [GO:0141113] (biological process) Relationships: is a type of GO:2000051; is a type of regulation of Wnt signaling pathway, planar cell polarity pathway [GO:2000095]; negatively regulates Wnt signaling pathway, planar cell polarity pathway [GO:0060071] Definition: Any process that stops, prevents, or reduces the frequency, rate or extent of the Wnt signaling pathway, planar cell polarity pathway. References: PMID:19056682